negative regulation of myosin II filament assembly [GO:1905510] (biological process) Note: positive regulation / down regulation of the formation of a bipolar filament composed of myosin II molecules Relationships: is a type of GO:0031333; is a type of regulation of myosin II filament assembly [GO:0043520]; is a type of negative regulation of myosin II filament organization [GO:1904900]; negatively regulates myosin II filament assembly [GO:0031036] Also known as: down regulation of myosin II filament assembly, down-regulation of myosin II filament assembly, downregulation of myosin II filament assembly, inhibition of myosin II filament assembly, down regulation of myosin II polymerization, down-regulation of myosin II polymerization, downregulation of myosin II polymerization, inhibition of myosin II polymerization, negative regulation of myosin II polymerization Definition: Any process that stops, prevents or reduces the frequency, rate or extent of myosin II filament assembly. References: PMID:27237792, PMID:7691416 Sources: GOC:TermGenie, GO_REF:0000058